ductus venosus closure [GO:0061116] (biological process) Relationships: is a type of venous blood vessel morphogenesis [GO:0048845] Sources: GOC:dph Definition: The morphogenesis process in which the ductus venosus changes to no longer permit blood flow after birth.